{
  "gene_symbol": "CD226",
  "term_id": "GO:0050862",
  "gene_name": "CD226 antigen",
  "gene": "UniProtKB:Q15762",
  "term_label": "positive regulation of T cell receptor signaling pathway"
}